{
  "gene_name": "Patched domain-containing protein 3",
  "term_label": "Unknown biological process",
  "gene_symbol": "PTCHD3",
  "term_id": "UNKNOWN:0002",
  "gene": "UniProtKB:Q3KNS1"
}